{
  "term_label": "Unknown cellular component",
  "gene_name": "Testis-expressed protein 45",
  "gene": "UniProtKB:Q8NA69",
  "term_id": "UNKNOWN:0003",
  "gene_symbol": "TEX45"
}